{
  "gene": "UniProtKB:Q13671",
  "gene_symbol": "RIN1",
  "term_id": "UNKNOWN:0002",
  "term_label": "Unknown biological process",
  "gene_name": "Ras and Rab interactor 1"
}